{
  "term_label": "polyubiquitin modification-dependent protein binding",
  "gene_name": "Large proline-rich protein BAG6",
  "gene_symbol": "BAG6",
  "gene": "UniProtKB:P46379",
  "term_id": "GO:0031593"
}